galactosyldiacylglycerol alpha-2,3-sialyltransferase activity [GO:0047289] (MF) Sources: EC:2.4.3.5 Definition: Catalysis of the reaction: 1,2-diacyl-3-beta-D-galactosyl-sn-glycerol + CMP-N-acetyl-beta-neuraminate = 1,2-diacyl-3-[3-(alpha-D-N-acetylneuraminyl)-beta-D-galactosyl]-sn-glycerol + CMP + H+. Relationships: is a type of GO:0008373